positive regulation of B cell deletion [GO:0002869] (biological process) Also known as: positive regulation of B lymphocyte deletion, positive regulation of B-cell deletion, positive regulation of B-lymphocyte deletion, up regulation of B cell deletion, up-regulation of B cell deletion, upregulation of B cell deletion, activation of B cell deletion, stimulation of B cell deletion Definition: Any process that activates or increases the frequency, rate, or extent of B cell deletion. Subtypes: positive regulation of central B cell deletion [GO:0002900], positive regulation of peripheral B cell deletion [GO:0002910] Sources: GOC:add Relationships: is a type of positive regulation of B cell tolerance induction [GO:0002663]; is a type of regulation of acute inflammatory response [GO:0002673]; is a type of regulation of B cell deletion [GO:0002867]; is_a positive regulation of B cell apoptotic process [GO:0002904]; is a type of positive regulation of apoptotic process involved in development [GO:1904747]; RO_0002213 GO:0002516